{
  "term_label": "plasma membrane",
  "gene_name": "Sulfate transporter",
  "gene_symbol": "SLC26A2",
  "term_id": "GO:0005886",
  "gene": "UniProtKB:P50443"
}